inositol-1,3,4,5-tetrakisphosphate 3-phosphatase activity [GO:0051717] (molecular function) Also known as: inositol (1,3,4,5)-tetrakisphosphate 3-phosphatase activity, inositol 1,3,4,5-tetrakisphosphate 3-phosphomonoesterase activity, inositol 1,3,4,5-tetrakisphosphate-5-phosphomonoesterase activity Sources: RHEA:77155 Relationships: is a type of inositol tetrakisphosphate phosphatase activity [GO:0052743] Definition: Catalysis of the reaction: 1D-myo-inositol 1,3,4,5-tetrakisphosphate + H2O = 1D-myo-inositol 1,4,5-trisphosphate + phosphate.